{
  "gene_symbol": "KLHL12",
  "term_label": "COPII vesicle coating",
  "gene": "UniProtKB:Q53G59",
  "term_id": "GO:0048208",
  "gene_name": "Kelch-like protein 12"
}